{
  "gene_name": "Decorin",
  "gene_symbol": "DCN",
  "term_id": "UNKNOWN:0001",
  "gene": "UniProtKB:P07585",
  "term_label": "Unknown molecular function"
}